genital disc pattern formation [GO:0035221] (biological process) Relationships: is a type of imaginal disc pattern formation [GO:0007447]; is part of genital disc development [GO:0035215] Sources: GOC:bf Subtypes: genital disc anterior/posterior pattern formation [GO:0035224] Definition: The process that gives rise to the patterns of cell differentiation that will arise in the genital imaginal disc.